{
  "gene_name": "Transmembrane channel-like protein 8",
  "term_id": "UNKNOWN:0003",
  "gene_symbol": "TMC8",
  "gene": "UniProtKB:Q8IU68",
  "term_label": "Unknown cellular component"
}